peroxisome organization [GO:0007031] (biological process) Definition: A process that is carried out at the cellular level which results in the assembly, arrangement of constituent parts, or disassembly of a peroxisome. A peroxisome is a small, membrane-bounded organelle that uses dioxygen (O2) to oxidize organic molecules. Sources: GOC:mah Also known as: peroxisome organisation, peroxisome organization and biogenesis Relationships: is_a organelle organization [GO:0006996] Subtypes: glyoxysome organization [GO:0010111], GO:0019817, ER-dependent peroxisome organization [GO:0032581], peroxisome inheritance [GO:0045033], protein localization to peroxisome [GO:0072662] Regulation: regulated by regulation of peroxisome organization [GO:1900063]; positively regulated by positive regulation of peroxisome organization [GO:1900064]